carotenoid catabolic process [GO:0016118] (biological process) Subtypes: xanthophyll catabolic process [GO:0016124], beta-carotene catabolic process [GO:1901811], beta-zeacarotene catabolic process [GO:1901817], alpha-zeacarotene catabolic process [GO:1901820], delta-carotene catabolic process [GO:1901823], zeaxanthin bis(beta-D-glucoside) catabolic process [GO:1901829] Also known as: carotenoid breakdown, carotenoid catabolism, carotenoid degradation Relationships: is a type of tetraterpenoid catabolic process [GO:0016110]; is_a carotenoid metabolic process [GO:0016116] Definition: The chemical reactions and pathways resulting in the breakdown of carotenoids, tetraterpenoid compounds in which two units of 4 isoprenoid residues joined head-to-tail are themselves joined tail-to-tail. Sources: GOC:go_curators